{
  "gene": "UniProtKB:Q99424",
  "term_id": "GO:0120524",
  "term_label": "long-chain fatty acyl-CoA oxidase activity",
  "gene_name": "Peroxisomal acyl-coenzyme A oxidase 2",
  "gene_symbol": "ACOX2"
}